{
  "gene_symbol": "STAM2",
  "term_label": "Unknown molecular function",
  "gene_name": "Signal transducing adapter molecule 2",
  "term_id": "UNKNOWN:0001",
  "gene": "UniProtKB:O75886"
}